{
  "gene_name": "Calcium-activated potassium channel subunit alpha-1",
  "term_id": "GO:0045211",
  "gene": "UniProtKB:Q12791",
  "term_label": "postsynaptic membrane",
  "gene_symbol": "KCNMA1"
}